{
  "gene_symbol": "PPP1CB",
  "gene_name": "Serine_threonine-protein phosphatase PP1-beta catalytic subunit",
  "term_label": "cytoplasm",
  "gene": "UniProtKB:P62140",
  "term_id": "GO:0005737"
}